Purkinje myocyte action potential [GO:0086017] (biological process) Sources: GOC:BHF, GOC:mtg_cardiac_conduct_nov11 Definition: An action potential that occurs in a Purkinje myocyte. Regulation: regulated by GO:0098906 Relationships: is a type of cardiac muscle cell action potential [GO:0086001]; is part of Purkinje myocyte to ventricular cardiac muscle cell signaling [GO:0086029]